{
  "term_label": "Unknown biological process",
  "gene_name": "Leucine-rich repeat-containing protein 42",
  "gene": "UniProtKB:Q9Y546",
  "gene_symbol": "LRRC42",
  "term_id": "UNKNOWN:0002"
}